{
  "term_label": "nucleolus",
  "gene": "UniProtKB:Q9H5U6",
  "gene_symbol": "ZCCHC4",
  "gene_name": "rRNA N6-adenosine-methyltransferase ZCCHC4",
  "term_id": "GO:0005730"
}